hyperpolarization of postsynaptic membrane [GO:0098818] (biological process) Sources: GOC:dos Relationships: is a type of GO:0060078 Definition: A process that hyerpolarizes a postsynaptic membrane relative to its resting potential. This has an inhibitory effect on the post-synaptic cell, moving the membrane potential away from the firing threshold.